response to sulfur dioxide [GO:0010477] (biological process) References: PMID:17425719 Subtypes: GO:0071252 Relationships: is a type of GO:1901700 Definition: Any process that results in a change in state or activity of a cell or an organism (in terms of movement, secretion, enzyme production, gene expression, etc.) as a result of a sulfur dioxide (SO2) stimulus.